central nervous system morphogenesis [GO:0021551] (biological process) Relationships: is a type of anatomical structure morphogenesis [GO:0009653]; is part of central nervous system development [GO:0007417] Definition: The process in which the anatomical structure of the central nervous system is generated and organized. The central nervous system is the core nervous system that serves an integrating and coordinating function. In vertebrates it consists of the brain and spinal cord. In those invertebrates with a central nervous system it typically consists of a brain, cerebral ganglia and a nerve cord. Sources: GOC:cls, GOC:dgh, GOC:dph, GOC:jid, GO_REF:0000021